{
  "gene": "UniProtKB:Q6ZRV2",
  "term_id": "GO:0044380",
  "term_label": "protein localization to cytoskeleton",
  "gene_symbol": "FAM83H",
  "gene_name": "Protein FAM83H"
}